nitrate reductase activity [GO:0008940] (molecular function) Relationships: is a type of oxidoreductase activity, acting on other nitrogenous compounds as donors [GO:0016661] Definition: Catalysis of the reaction: nitrite + acceptor = nitrate + reduced acceptor. Subtypes: ferredoxin-nitrate reductase activity [GO:0047889], nitrate reductase (cytochrome) activity [GO:0050140], GO:0050463, nitrate reductase (quinone) activity [GO:0160182] Sources: RHEA:21068 Also known as: respiratory nitrate reductase activity, nitrate reductase (acceptor), nitrite:(acceptor) oxidoreductase, nitrite:acceptor oxidoreductase